{
  "term_id": "UNKNOWN:0002",
  "term_label": "Unknown biological process",
  "gene_symbol": "IQCF5",
  "gene": "UniProtKB:A8MTL0",
  "gene_name": "IQ domain-containing protein F5"
}